2,6-dihydroxypyridine 3-monooxygenase activity [GO:0018663] (molecular function) Also known as: 2,6-dihydroxypyridine oxidase activity, 2,6-dihydroxypyridine,NADH:oxygen oxidoreductase (3-hydroxylating) Relationships: is_a oxidoreductase activity, acting on paired donors, with incorporation or reduction of molecular oxygen, NAD(P)H as one donor, and incorporation of one atom of oxygen [GO:0016709] Definition: Catalysis of the reaction: 2,6-dihydroxypyridine + H+ + NADH + O2 = 2,3,6-trihydroxypyridine + H2O + NAD+. Sources: EC:1.14.13.10, RHEA:16917